{
  "term_id": "UNKNOWN:0001",
  "term_label": "Unknown molecular function",
  "gene_symbol": "YWHAB",
  "gene_name": "14-3-3 protein beta_alpha",
  "gene": "UniProtKB:P31946"
}